{
  "gene": "UniProtKB:Q15486",
  "term_id": "UNKNOWN:0001",
  "gene_name": "Putative inactive beta-glucuronidase-like protein SMA3",
  "gene_symbol": "GUSBP1",
  "term_label": "Unknown molecular function"
}